compound leaf morphogenesis [GO:0060777] (biological process) Relationships: is a type of GO:0009965 Definition: The leaf morphogenesis process that results in the shaping of a compound leaf. A compound leaf is a leaf having two or more distinct leaflets that are evident as such from early in development. Sources: GOC:dph, GOC:sdb_2009, GOC:tb